{
  "term_label": "protein methyltransferase activity",
  "gene_symbol": "HEMK2",
  "gene_name": "Methyltransferase N6AMT1",
  "gene": "UniProtKB:Q9Y5N5",
  "term_id": "GO:0008276"
}